{
  "term_label": "receptor complex",
  "gene_symbol": "ROR1",
  "gene": "UniProtKB:Q01973",
  "gene_name": "Inactive tyrosine-protein kinase transmembrane receptor ROR1",
  "term_id": "GO:0043235"
}